{
  "gene_name": "CD180 antigen",
  "term_label": "plasma membrane",
  "term_id": "GO:0005886",
  "gene_symbol": "CD180",
  "gene": "UniProtKB:Q99467"
}